symbiont-mediated modulation of host virulence [GO:0098676] (BP) Relationships: is_a symbiont-mediated perturbation of host process [GO:0044003] References: PMID:10913072, PMID:11553559, PMID:22919604, PMID:8658163 Sources: VZ:3965 Definition: A process by which a virus improves the virulence of its host for that host's respective host. Common in but not limited to bacteriophages; also occurs in phage-bearing bacteria infecting plants or animals for example. Mechanisms include the expression of factors that modulate a bacterial adhesion to a host cell, spread through host tissues, production of exotoxins or provide protection against host immune defenses. Also known as: modulation of host virulence by virus